phosphatidylinositol transfer activity [GO:0008526] (molecular function) Relationships: is_a phospholipid transfer activity [GO:0120014]; has part phosphatidylinositol binding [GO:0035091] Also known as: phosphatidylinositol transporter activity, phosphatidylinositol carrier activity, intermembrane phosphatidylinositol transfer activity, intermembrane phosphotidylinositol transfer activity References: PMID:20823909, PMID:24220498, PMID:25797198 Sources: GOC:krc Definition: Removes phosphatidylinositol from a membrane or a monolayer lipid particle, transports it through the aqueous phase while protected in a hydrophobic pocket, and brings it to an acceptor membrane or lipid particle. Subtypes: phosphatidylserine-phosphatidylinositol-4-phosphate exchange activity [GO:0160270], GO:0160291